{
  "term_label": "Unknown cellular component",
  "term_id": "UNKNOWN:0003",
  "gene_symbol": "ENPP5",
  "gene": "UniProtKB:Q9UJA9",
  "gene_name": "Ectonucleotide pyrophosphatase_phosphodiesterase family member 5"
}